{
  "term_id": "GO:0042633",
  "gene": "UniProtKB:Q9BYQ8",
  "term_label": "hair cycle",
  "gene_name": "Keratin-associated protein 4-9",
  "gene_symbol": "KRTAP4-9"
}